{
  "gene": "UniProtKB:O95741",
  "gene_name": "Copine-6",
  "gene_symbol": "CPNE6",
  "term_label": "calcium-dependent phospholipid binding",
  "term_id": "GO:0005544"
}